negative regulation of receptor signaling pathway via STAT [GO:1904893] (biological process) Relationships: is a type of negative regulation of signal transduction [GO:0009968]; is a type of regulation of receptor signaling pathway via STAT [GO:1904892]; negatively regulates cell surface receptor signaling pathway via STAT [GO:0097696] Also known as: down regulation of STAT cascade, down regulation of STAT signalling pathway, down regulation of kinase activated-STAT cascade, down regulation of kinase-STAT cascade, down-regulation of STAT cascade, down-regulation of STAT signalling pathway, down-regulation of kinase activated-STAT cascade, down-regulation of kinase-STAT cascade, downregulation of STAT cascade, downregulation of STAT signalling pathway, downregulation of kinase activated-STAT cascade, downregulation of kinase-STAT cascade, negative regulation of STAT signalling pathway, negative regulation of kinase activated-STAT cascade, negative regulation of kinase-STAT cascade, inhibition of STAT cascade, inhibition of STAT signalling pathway, inhibition of kinase activated-STAT cascade, inhibition of kinase-STAT cascade Definition: Any process that stops, prevents or reduces the frequency, rate or extent of receptor signaling via STAT. References: PMID:24587195 Sources: GOC:TermGenie, GOC:rjd, GO_REF:0000058 Subtypes: negative regulation of receptor signaling pathway via JAK-STAT [GO:0046426]